{
  "term_label": "positive regulation of protein localization to spindle pole body",
  "gene_symbol": "NUMA1",
  "gene": "UniProtKB:Q14980",
  "gene_name": "Nuclear mitotic apparatus protein 1",
  "term_id": "GO:1902365"
}